{
  "gene_name": "C-type lectin domain family 7 member A",
  "gene": "UniProtKB:Q9BXN2",
  "term_id": "GO:0001872",
  "term_label": "(1->3)-beta-D-glucan binding",
  "gene_symbol": "CLEC7A"
}